{
  "gene": "UniProtKB:P05141",
  "gene_symbol": "SLC25A5",
  "term_id": "GO:0005471",
  "term_label": "ATP:ADP antiporter activity",
  "gene_name": "ADP_ATP translocase 2"
}